{
  "term_label": "phosphatidylinositol bisphosphate binding",
  "gene": "UniProtKB:P12271",
  "gene_name": "Retinaldehyde-binding protein 1",
  "gene_symbol": "RLBP1",
  "term_id": "GO:1902936"
}